{
  "gene": "UniProtKB:P82909",
  "term_label": "Unknown molecular function",
  "gene_symbol": "KGD4",
  "term_id": "UNKNOWN:0001",
  "gene_name": "Alpha-ketoglutarate dehydrogenase component 4"
}